regulation of establishment or maintenance of cell polarity [GO:0032878] (biological process) Definition: Any process that modulates the frequency, rate or extent of the specification, formation or maintenance of anisotropic intracellular organization or cell growth patterns. Sources: GOC:mah Relationships: is_a regulation of cellular process [GO:0050794]; RO_0002211 GO:0007163 Subtypes: regulation of cytoskeleton polarization involved in growth plate cartilage chondrocyte division [GO:0003427], regulation of establishment or maintenance of bipolar cell polarity [GO:2000099], regulation of establishment of cell polarity [GO:2000114], negative regulation of establishment or maintenance of neuroblast polarity [GO:2000248], regulation of establishment or maintenance of cell polarity regulating cell shape [GO:2000769]